3',5'-cGMP-stimulated cyclic-nucleotide phosphodiesterase activity [GO:0004118] (molecular function) Note: cGMP-stimulated cyclic-nucleotide phosphodiesterase activity Relationships: is a type of 3',5'-cyclic-nucleotide phosphodiesterase activity [GO:0004114] Definition: Catalysis of the reaction: nucleoside 3',5'-cyclic phosphate + H2O = nucleoside 5'-phosphate; catalytic activity is increased in the presence of cGMP. References: PMID:15210692, PMID:35216259 Sources: GOC:mah